{
  "gene_symbol": "SMC6",
  "term_label": "single-stranded DNA binding",
  "gene_name": "Structural maintenance of chromosomes protein 6",
  "gene": "UniProtKB:Q96SB8",
  "term_id": "GO:0003697"
}